(R)-4-hydroxymandelate catabolic process [GO:0019599] (BP) Definition: The chemical reactions and pathways resulting in the breakdown of (R)-4-hydroxymandelate, the anion of (R)-4-hydroxymandelic acid. Sources: GOC:ai Relationships: is a type of phenol-containing compound catabolic process [GO:0019336]; is a type of monocarboxylic acid catabolic process [GO:0072329] Also known as: (R)-4-hydroxymandelate breakdown, (R)-4-hydroxymandelate catabolism, (R)-4-hydroxymandelate degradation